regulation of glial cell differentiation [GO:0045685] (biological process) Relationships: is a type of regulation of cell differentiation [GO:0045595]; regulates GO:0010001 Also known as: regulation of glia cell differentiation, regulation of neuroglia differentiation Definition: Any process that modulates the frequency, rate or extent of glia cell differentiation. Sources: GOC:go_curators Subtypes: regulation of microglia differentiation [GO:0014006], regulation of Schwann cell differentiation [GO:0014038], GO:0045686, positive regulation of glial cell differentiation [GO:0045687], GO:0048710, GO:0048713